cinnamyl-alcohol dehydrogenase activity [GO:0045551] (molecular function) Definition: Catalysis of the reaction: cinnamyl alcohol + NADP+ = cinnamaldehyde + NADPH + H+. Also acts on coniferyl alcohol, sinapyl alcohol and 4-coumaryl alcohol. Sources: EC:1.1.1.195 Relationships: is a type of oxidoreductase activity, acting on the CH-OH group of donors, NAD or NADP as acceptor [GO:0016616] Also known as: CAD activity, cinnamyl alcohol dehydrogenase activity, cinnamyl-alcohol:NADP+ oxidoreductase activity